{
  "gene_name": "Neuromodulin",
  "gene_symbol": "GAP43",
  "term_label": "plasma membrane",
  "gene": "UniProtKB:P17677",
  "term_id": "GO:0005886"
}